{
  "gene_symbol": "CFAP221",
  "gene_name": "Cilia- and flagella-associated protein 221",
  "term_label": "9+2 motile cilium",
  "term_id": "GO:0097729",
  "gene": "UniProtKB:Q4G0U5"
}